{
  "gene_name": "Plectin",
  "term_label": "sarcolemma",
  "gene_symbol": "PLEC",
  "term_id": "GO:0042383",
  "gene": "UniProtKB:Q15149"
}